{
  "gene_symbol": "TAF1B",
  "term_label": "RNA polymerase I core promoter sequence-specific DNA binding",
  "term_id": "GO:0001164",
  "gene_name": "TATA box-binding protein-associated factor RNA polymerase I subunit B",
  "gene": "UniProtKB:Q53T94"
}